{
  "term_label": "Unknown cellular component",
  "gene_symbol": "OR5H2",
  "gene": "UniProtKB:Q8NGV7",
  "term_id": "UNKNOWN:0003",
  "gene_name": "Olfactory receptor 5H2"
}